{
  "gene_symbol": "CST5",
  "term_id": "GO:0004869",
  "gene_name": "Cystatin-D",
  "term_label": "cysteine-type endopeptidase inhibitor activity",
  "gene": "UniProtKB:P28325"
}